negative regulation of interleukin-20 production [GO:0032704] (biological process) Also known as: down regulation of interleukin-20 production, down-regulation of interleukin-20 production, downregulation of interleukin-20 production, negative regulation of IL-20 production, inhibition of interleukin-20 production, negative regulation of interleukin-20 biosynthetic process Relationships: is_a GO:0001818; is a type of GO:0032664; negatively regulates GO:0032624 Definition: Any process that stops, prevents, or reduces the frequency, rate, or extent of interleukin-20 production. Sources: GOC:mah